{
  "gene": "UniProtKB:Q16656",
  "term_label": "DNA-binding transcription factor activity, RNA polymerase II-specific",
  "gene_name": "Nuclear respiratory factor 1",
  "term_id": "GO:0000981",
  "gene_symbol": "NRF1"
}